{
  "gene_symbol": "IGHV3-7",
  "gene_name": "Immunoglobulin heavy variable 3-7",
  "term_label": "immunoglobulin mediated immune response",
  "term_id": "GO:0016064",
  "gene": "UniProtKB:P01780"
}